positive regulation of mitotic cell cycle [GO:0045931] (biological process) Relationships: is a type of regulation of mitotic cell cycle [GO:0007346]; is a type of positive regulation of cell cycle [GO:0045787]; RO_0002213 mitotic cell cycle [GO:0000278] Subtypes: positive regulation of mitotic cell cycle, embryonic [GO:0045977], positive regulation of mitotic spindle organization [GO:0110028], negative regulation of cell cycle switching, mitotic to meiotic cell cycle [GO:0110045], positive regulation of mitotic cell cycle phase transition [GO:1901992], positive regulation of mitotic cell cycle DNA replication [GO:1903465], negative regulation of mitotic DNA damage checkpoint [GO:1904290] Definition: Any process that activates or increases the rate or extent of progression through the mitotic cell cycle. Also known as: positive regulation of mitotic cell cycle progression, positive regulation of progression through mitotic cell cycle, up regulation of progression through mitotic cell cycle, up-regulation of progression through mitotic cell cycle, upregulation of progression through mitotic cell cycle, activation of progression through mitotic cell cycle, stimulation of progression through mitotic cell cycle Sources: GOC:dph, GOC:go_curators, GOC:tb